{
  "gene_symbol": "OR8K1",
  "term_label": "Unknown molecular function",
  "gene": "UniProtKB:Q8NGG5",
  "gene_name": "Olfactory receptor 8K1",
  "term_id": "UNKNOWN:0001"
}